melanocortin receptor binding [GO:0031779] (molecular function) Relationships: is a type of GO:0071855 Definition: Binding to a melanocortin receptor. Subtypes: corticotropin hormone receptor binding [GO:0031780], type 3 melanocortin receptor binding [GO:0031781], GO:0031782, type 5 melanocortin receptor binding [GO:0031783], type 1 melanocortin receptor binding [GO:0070996] Also known as: melanocortin receptor ligand Sources: GOC:mah, GOC:nln